{
  "gene": "UniProtKB:A4D2B0",
  "gene_symbol": "MBLAC1",
  "gene_name": "Metallo-beta-lactamase domain-containing protein 1",
  "term_label": "Unknown molecular function",
  "term_id": "UNKNOWN:0001"
}